posterior Malpighian tubule development [GO:0061328] (biological process) Definition: The process whose specific outcome is the progression of the posterior Malpighian tubule over time, from its formation to the mature structure. The pair of posterior tubules arise from a ventrolateral region of the embryonic hindgut and project backwards through the body cavity. A Malpighian tubule is a fine, thin-walled excretory tubule in insects which connects with the posterior part of the gut. Relationships: is a type of Malpighian tubule development [GO:0072002] Sources: GOC:dph, GOC:mtg_kidney_jan10